{
  "term_id": "GO:0008543",
  "gene_name": "Fibroblast growth factor 1",
  "term_label": "fibroblast growth factor receptor signaling pathway",
  "gene": "UniProtKB:P05230",
  "gene_symbol": "FGF1"
}